{
  "term_id": "GO:0000423",
  "term_label": "mitophagy",
  "gene": "UniProtKB:Q9H492",
  "gene_name": "Microtubule-associated proteins 1A_1B light chain 3A",
  "gene_symbol": "MAP1LC3A"
}